{
  "gene_symbol": "NAT10",
  "term_id": "GO:0002101",
  "term_label": "tRNA wobble cytosine modification",
  "gene_name": "RNA cytidine acetyltransferase",
  "gene": "UniProtKB:Q9H0A0"
}